TRAIL binding [GO:0045569] (molecular function) Also known as: Apo-2L binding Relationships: is a type of protein binding [GO:0005515] References: PMID:9082980 Sources: GOC:go_curators Definition: Binding to TRAIL (TNF-related apoptosis inducing ligand), a member of the tumor necrosis factor ligand family that rapidly induces apoptosis in a variety of transformed cell lines.